{
  "term_label": "neuronal cell body",
  "gene_name": "Ermin",
  "gene_symbol": "ERMN",
  "term_id": "GO:0043025",
  "gene": "UniProtKB:Q8TAM6"
}